{
  "gene_symbol": "H2AC19",
  "term_label": "heterochromatin formation",
  "gene": "UniProtKB:Q6FI13",
  "term_id": "GO:0031507",
  "gene_name": "Histone H2A type 2-A"
}